{
  "gene": "UniProtKB:P31512",
  "gene_symbol": "FMO4",
  "term_id": "GO:0006805",
  "gene_name": "Dimethylaniline monooxygenase [N-oxide-forming] 4",
  "term_label": "xenobiotic metabolic process"
}